cerebellar granule cell to Purkinje cell synapse [GO:0150048] (cellular component) References: PMID:12427822 Sources: GOC:aruk, GOC:bc Definition: A synapse of a granule cell fiber onto the dendrites of a Purkinje cell in cerebellum. Also known as: cerebellar parallel fiber to Purkinje cell synapse Relationships: is a type of asymmetric, glutamatergic, excitatory synapse [GO:0098985]